{
  "term_id": "GO:0005813",
  "term_label": "centrosome",
  "gene_name": "SAC3 domain-containing protein 1",
  "gene_symbol": "SAC3D1",
  "gene": "UniProtKB:A6NKF1"
}